{
  "gene": "UniProtKB:O94925",
  "gene_name": "Glutaminase kidney isoform, mitochondrial",
  "gene_symbol": "GLS",
  "term_label": "glutaminase activity",
  "term_id": "GO:0004359"
}